dolichyl pyrophosphate Man9GlcNAc2 alpha-1,3-glucosyltransferase activity [GO:0042281] (molecular function) Relationships: is a type of GO:0004583; is part of dolichol-linked oligosaccharide biosynthetic process [GO:0006488] Definition: Catalysis of the addition of the first glucose residue to the lipid-linked oligosaccharide precursor for N-linked glycosylation; the transfer of glucose from dolichyl phosphate glucose (Dol-P-Glc) on to the lipid-linked oligosaccharide Man(9)GlcNAc(2)-PP-Dol. Sources: GOC:al, MetaCyc:RXN-5470 Also known as: dolichyl-P-Glc:Man9GlcNAc2-PP-dolichyl glucosyltransferase activity